{
  "gene_symbol": "DOCK8",
  "term_id": "GO:2000406",
  "term_label": "positive regulation of T cell migration",
  "gene": "UniProtKB:Q8NF50",
  "gene_name": "Dedicator of cytokinesis protein 8"
}